shoot regeneration [GO:0062210] (biological process) Relationships: is a type of GO:0031099; is_a GO:0048367 References: PMID:27143753 Definition: The regeneration process by which a damaged or lost shoot regrows or re-differentiates. This process may occur via de-differentiation and subsequent reprogramming of somatic cells or activation of existing undifferentiated (meristematic) cells to produce a new shoot meristem and subsequently a new shoot. Also known as: shoot system regeneration